cell wall modification involved in fruit ripening [GO:0009829] (biological process) Also known as: cell wall modification during ripening Relationships: is a type of GO:0009827; is a type of cellular process involved in reproduction in multicellular organism [GO:0022412]; BFO_0000050 fruit ripening [GO:0009835] Definition: The series of events resulting in chemical or structural alterations of existing cell walls that contribute to fruit ripening. Sources: GOC:lr